{
  "gene_name": "General transcription factor IIH subunit 2-like protein",
  "term_label": "Unknown molecular function",
  "gene_symbol": "GTF2H2C",
  "gene": "UniProtKB:Q6P1K8",
  "term_id": "UNKNOWN:0001"
}